{
  "term_id": "GO:0000981",
  "term_label": "DNA-binding transcription factor activity, RNA polymerase II-specific",
  "gene": "UniProtKB:Q8N2I2",
  "gene_name": "Zinc finger protein 619",
  "gene_symbol": "ZNF619"
}